{
  "gene_symbol": "CRELD1",
  "term_id": "UNKNOWN:0002",
  "gene_name": "Protein disulfide isomerase CRELD1",
  "gene": "UniProtKB:Q96HD1",
  "term_label": "Unknown biological process"
}